negative gravitropism [GO:0009959] (biological process) Also known as: shoot gravitropism Sources: GOC:sm Relationships: is_a gravitropism [GO:0009630] Definition: The orientation of plant parts away from gravity.